{
  "term_id": "UNKNOWN:0003",
  "term_label": "Unknown cellular component",
  "gene": "UniProtKB:Q9BYP8",
  "gene_name": "Keratin-associated protein 17-1",
  "gene_symbol": "KRTAP17-1"
}